peripheral nervous system myelin maintenance [GO:0032287] (biological process) Relationships: is a type of myelin maintenance [GO:0043217]; is part of GO:0022011 Sources: GOC:dgh Also known as: myelin maintenance in peripheral nervous system, peripheral nervous system myelin sheath maintenance Definition: The process in which the structure and material content of mature peripheral nervous system myelin is kept in a functional state.